{
  "gene_symbol": "NOBOX",
  "term_id": "UNKNOWN:0003",
  "gene": "UniProtKB:O60393",
  "term_label": "Unknown cellular component",
  "gene_name": "Homeobox protein NOBOX"
}